epithelial cell maturation involved in salivary gland development [GO:0060691] (biological process) Sources: GOC:dph Relationships: is_a epithelial cell maturation [GO:0002070]; is part of epithelial cell differentiation involved in salivary gland development [GO:0060690] Definition: The developmental process, independent of morphogenetic (shape) change, that is required for an epithelial cell of the salivary gland to attain its fully functional state.